{
  "term_id": "GO:0005615",
  "gene": "UniProtKB:O76096",
  "term_label": "extracellular space",
  "gene_name": "Cystatin-F",
  "gene_symbol": "CST7"
}